{
  "gene_symbol": "PRR14",
  "gene": "UniProtKB:Q9BWN1",
  "term_id": "UNKNOWN:0002",
  "term_label": "Unknown biological process",
  "gene_name": "Proline-rich protein 14"
}